{
  "term_label": "angiogenesis",
  "gene_name": "Cell surface glycoprotein MUC18",
  "gene": "UniProtKB:P43121",
  "gene_symbol": "MCAM",
  "term_id": "GO:0001525"
}